{
  "gene_name": "Tripartite motif-containing protein 46",
  "term_id": "GO:0044304",
  "gene_symbol": "TRIM46",
  "gene": "UniProtKB:Q7Z4K8",
  "term_label": "main axon"
}